{
  "term_label": "D-serine biosynthetic process",
  "gene": "UniProtKB:Q9GZT4",
  "gene_name": "Serine racemase",
  "gene_symbol": "SRR",
  "term_id": "GO:0070179"
}